{
  "gene_symbol": "UHMK1",
  "gene": "UniProtKB:Q8TAS1",
  "term_id": "GO:0045948",
  "gene_name": "Serine_threonine-protein kinase Kist",
  "term_label": "positive regulation of translational initiation"
}